{
  "gene_symbol": "PLK2",
  "term_id": "GO:0005634",
  "term_label": "nucleus",
  "gene_name": "Serine_threonine-protein kinase PLK2",
  "gene": "UniProtKB:Q9NYY3"
}